{
  "gene_name": "Protein FAM161A",
  "term_label": "photoreceptor connecting cilium",
  "term_id": "GO:0032391",
  "gene": "UniProtKB:Q3B820",
  "gene_symbol": "FAM161A"
}